{
  "gene": "UniProtKB:A0A075B6X5",
  "term_label": "adaptive immune response",
  "term_id": "GO:0002250",
  "gene_symbol": "TRAV18",
  "gene_name": "T cell receptor alpha variable 18"
}